{
  "term_id": "GO:0006515",
  "gene_name": "LON peptidase N-terminal domain and RING finger protein 2",
  "gene": "UniProtKB:Q1L5Z9",
  "gene_symbol": "LONRF2",
  "term_label": "protein quality control for misfolded or incompletely synthesized proteins"
}